{
  "term_label": "nuclear export",
  "gene": "UniProtKB:Q99666",
  "gene_name": "RANBP2-like and GRIP domain-containing protein 5_6",
  "gene_symbol": "RGPD5",
  "term_id": "GO:0051168"
}